basal body patch [GO:0120220] (cellular component) Definition: The region in the apical portion of multiciliated epithelial cells where the ciliary basal bodies cluster. Relationships: is a type of cellular anatomical structure [GO:0110165]; is part of apical part of cell [GO:0045177] Also known as: centriolar patch References: PMID:20164345, PMID:20685736, PMID:29891944 Sources: GOC:krc